2-isopropylphenol monooxygenase activity [GO:0102323] (molecular function) Definition: Catalysis of the reaction: 2-isopropylphenol + O2 + NADH + H+ = 3-isopropylcatechol + H2O + NAD. Relationships: is a type of oxidoreductase activity, acting on paired donors, with incorporation or reduction of molecular oxygen, NAD(P)H as one donor, and incorporation of one atom of oxygen [GO:0016709] Sources: GOC:pz, RHEA:63520